{
  "gene_symbol": "HLA-DRA",
  "gene_name": "HLA class II histocompatibility antigen, DR alpha chain",
  "gene": "UniProtKB:P01903",
  "term_id": "GO:0042613",
  "term_label": "MHC class II protein complex"
}